{
  "term_id": "UNKNOWN:0003",
  "gene_name": "Olfactory receptor 8H3",
  "gene": "UniProtKB:Q8N146",
  "gene_symbol": "OR8H3",
  "term_label": "Unknown cellular component"
}